{
  "term_id": "UNKNOWN:0002",
  "term_label": "Unknown biological process",
  "gene": "UniProtKB:O00461",
  "gene_symbol": "GOLIM4",
  "gene_name": "Golgi integral membrane protein 4"
}